NVT complex [GO:0061957] (cellular component) Relationships: is a type of protein-containing complex [GO:0032991] Definition: A protein complex that is capable of contributing to protein localization by the NVT pathway. In fission yeast, the Nvt complex consists of Ape2, Lap2 and Nbr1. References: PMID:26365378